{
  "gene_name": "Stress-70 protein, mitochondrial",
  "gene_symbol": "HSPA9",
  "term_label": "mitochondrion",
  "gene": "UniProtKB:P38646",
  "term_id": "GO:0005739"
}